{
  "gene_name": "Beta-1,4-galactosyltransferase 4",
  "gene_symbol": "B4GALT4",
  "term_label": "Golgi apparatus",
  "gene": "UniProtKB:O60513",
  "term_id": "GO:0005794"
}